{
  "term_label": "flavone metabolic process",
  "gene": "UniProtKB:Q9HAW9",
  "gene_name": "UDP-glucuronosyltransferase 1A8",
  "gene_symbol": "UGT1A8",
  "term_id": "GO:0051552"
}